{
  "gene": "UniProtKB:Q9Y5Y7",
  "gene_name": "Lymphatic vessel endothelial hyaluronic acid receptor 1",
  "term_id": "UNKNOWN:0002",
  "term_label": "Unknown biological process",
  "gene_symbol": "LYVE1"
}